protein-DNA complex organization [GO:0071824] (biological process) Definition: Any process in which macromolecules aggregate, disaggregate, or are modified, resulting in the formation, disassembly, or alteration of a protein-DNA complex. Sources: GOC:mah Also known as: DNA-protein complex subunit organization, protein-DNA complex subunit organisation, protein-DNA complex subunit organization Relationships: is a type of protein-containing complex organization [GO:0043933] Subtypes: protein-DNA complex remodeling [GO:0001120], GO:0032986, GO:0034728, GO:0065004